{
  "gene_name": "BPI fold-containing family A member 1",
  "gene_symbol": "BPIFA1",
  "term_label": "antimicrobial humoral immune response mediated by antimicrobial peptide",
  "term_id": "GO:0061844",
  "gene": "UniProtKB:Q9NP55"
}